{
  "gene": "UniProtKB:P09884",
  "gene_symbol": "POLA1",
  "term_label": "single-stranded DNA binding",
  "term_id": "GO:0003697",
  "gene_name": "DNA polymerase alpha catalytic subunit"
}